regulation of epithelial cell migration [GO:0010632] (biological process) Sources: GOC:BHF, GOC:dph, GOC:tb Definition: Any process that modulates the frequency, rate or extent of epithelial cell migration. Relationships: is a type of regulation of cell migration [GO:0030334]; is a type of regulation of multicellular organismal process [GO:0051239]; regulates GO:0010631 Subtypes: negative regulation of epithelial cell migration [GO:0010633], positive regulation of epithelial cell migration [GO:0010634], GO:0051547, regulation of border follicle cell migration [GO:1903684], regulation of epithelial cell migration, open tracheal system [GO:2000274]